{
  "gene_symbol": "CEBPB",
  "term_id": "GO:0006357",
  "gene_name": "CCAAT_enhancer-binding protein beta",
  "gene": "UniProtKB:P17676",
  "term_label": "regulation of transcription by RNA polymerase II"
}